brassinosteroid biosynthetic process [GO:0016132] (biological process) Relationships: is a type of GO:0016129; is a type of GO:0016131 Sources: ISBN:0192801023 Also known as: brassinosteroid anabolism, brassinosteroid biosynthesis, brassinosteroid formation, brassinosteroid synthesis Definition: The chemical reactions and pathways resulting in the formation of brassinosteroids, any of a group of steroid derivatives that occur at very low concentrations in plant tissues and may have hormone-like effects. Regulation: regulated by GO:0010422; negatively regulated by negative regulation of brassinosteroid biosynthetic process [GO:0010423]; positively regulated by positive regulation of brassinosteroid biosynthetic process [GO:2000488]